{
  "term_label": "insulin-responsive compartment",
  "gene": "UniProtKB:P61018",
  "term_id": "GO:0032593",
  "gene_symbol": "RAB4B",
  "gene_name": "Ras-related protein Rab-4B"
}